{
  "gene_name": "Unconventional myosin-VIIa",
  "term_label": "membrane",
  "gene": "UniProtKB:Q13402",
  "term_id": "GO:0016020",
  "gene_symbol": "MYO7A"
}